U12-type catalytic step 1 spliceosome [GO:0071017] (cellular component) Relationships: is a type of U12-type spliceosomal complex [GO:0005689]; is a type of GO:0071012; has part U6atac snRNP [GO:0005691]; has part GO:0005693 References: PMID:16201866 Sources: GOC:ab, GOC:krc, GOC:mah, ISBN:0879695897, ISBN:0879697393 Also known as: U12-type activated spliceosome, minor catalytic step 1 spliceosome, AT-AC catalytic step 1 spliceosome, mammalian U12-type spliceosomal complex B*, mammalian U12-type spliceosomal complex B2, yeast U12-type spliceosomal complex A1 Definition: A spliceosomal complex that is formed by the displacement of the U11 and U4atac snRNPs from the precatalytic spliceosome; the U12, U5 and U6atac snRNPs remain associated with the mRNA. This complex, sometimes called the activated spliceosome, is the catalytically active form of the spliceosome, and includes many proteins in addition to those found in the U12, and U5 and U6atac snRNPs.